{
  "gene_symbol": "SPTBN5",
  "gene": "UniProtKB:Q9NRC6",
  "term_label": "plasma membrane",
  "gene_name": "Spectrin beta chain, non-erythrocytic 5",
  "term_id": "GO:0005886"
}